cellular response to benzoic acid [GO:0071319] (biological process) Relationships: is a type of GO:0080021; is a type of cellular response to oxygen-containing compound [GO:1901701] Sources: GOC:mah Definition: Any process that results in a change in state or activity of a cell (in terms of movement, secretion, enzyme production, gene expression, etc.) as a result of a benzoic acid stimulus.